synaptic transmission, glycinergic [GO:0060012] (biological process) Definition: The vesicular release of glycine from a presynapse, across a chemical synapse, the subsequent activation of glycine receptors at the postsynapse of a target cell (neuron, muscle, or secretory cell) and the effects of this activation on the postsynaptic membrane potential and ionic composition of the postsynaptic cytosol. This process encompasses both spontaneous and evoked release of neurotransmitter and all parts of synaptic vesicle exocytosis. Evoked transmission starts with the arrival of an action potential at the presynapse. Regulation: regulated by regulation of synaptic transmission, glycinergic [GO:0060092]; negatively regulated by negative regulation of synaptic transmission, glycinergic [GO:0060093]; positively regulated by positive regulation of synaptic transmission, glycinergic [GO:0060094] Also known as: glycinergic synaptic transmission Sources: GOC:dos Relationships: is a type of GO:0007268